{
  "term_id": "GO:0005886",
  "gene_name": "Leucine-rich repeat neuronal protein 2",
  "gene_symbol": "LRRN2",
  "gene": "UniProtKB:O75325",
  "term_label": "plasma membrane"
}